ribonucleoside-diphosphate reductase inhibitor activity [GO:1990846] (molecular function) Relationships: is a type of enzyme inhibitor activity [GO:0004857]; negatively regulates ribonucleoside-diphosphate reductase activity [GO:0061731] Definition: Binds to and stops, prevents or reduces the activity of ribonucleoside-diphosphate reductase. References: PMID:16317005